{
  "gene": "UniProtKB:Q16613",
  "term_label": "aralkylamine N-acetyltransferase activity",
  "gene_symbol": "AANAT",
  "term_id": "GO:0004059",
  "gene_name": "Serotonin N-acetyltransferase"
}